amyloplast inner membrane [GO:0033098] (cellular component) Definition: The inner, i.e. lumen-facing, lipid bilayer of the amyloplast envelope; also faces the amyloplast stroma. Relationships: is a type of GO:0009528; is a type of amyloplast membrane [GO:0033097] Sources: GOC:ecd